vacuole-mitochondria membrane tethering [GO:0140057] (biological process) References: PMID:27875684 Relationships: is a type of organelle localization by membrane tethering [GO:0140056] Definition: The attachment of a mitochondrial membrane to a vacuolar membrane via molecular tethers that physically bridge their respective membranes and attach them to each other. The tethering may facilitate exchange of metabolites between the organelles.